{
  "gene_symbol": "FDXACB1",
  "gene": "UniProtKB:Q9BRP7",
  "term_label": "cytoplasm",
  "term_id": "GO:0005737",
  "gene_name": "Ferredoxin-fold anticodon-binding domain-containing protein 1"
}